{
  "term_id": "GO:0099171",
  "term_label": "presynaptic modulation of chemical synaptic transmission",
  "gene_name": "Neuronal acetylcholine receptor subunit alpha-5",
  "gene": "UniProtKB:P30532",
  "gene_symbol": "CHRNA5"
}